{
  "gene_name": "Alpha-ketoglutarate-dependent dioxygenase alkB homolog 3",
  "term_label": "mitochondrion",
  "term_id": "GO:0005739",
  "gene": "UniProtKB:Q96Q83",
  "gene_symbol": "ALKBH3"
}